{
  "term_id": "GO:0034198",
  "term_label": "cellular response to amino acid starvation",
  "gene_name": "GATOR complex protein NPRL3",
  "gene_symbol": "NPRL3",
  "gene": "UniProtKB:Q12980"
}